enoyl-[acyl-carrier-protein] reductase [NAD(P)H] activity [GO:0016631] (molecular function) Definition: Catalysis of the reaction: acyl-[acyl-carrier protein] + NAD(P)+ = trans-2,3-dehydroacyl-[acyl-carrier protein] + NAD(P)H + H+. Note: This term should not be used for direct annotation; please use of the children that specifies the cofactor of the reaction (NAD+ or NADP+): enoyl-[acyl-carrier-protein] reductase (NADH) activity ; GO:0004318 or enoyl-[acyl-carrier-protein] reductase (NADPH) activity ; GO:0141148. Relationships: is a type of oxidoreductase activity, acting on the CH-CH group of donors, NAD or NADP as acceptor [GO:0016628] Subtypes: enoyl-[acyl-carrier-protein] reductase (NADH) activity [GO:0004318], enoyl-[acyl-carrier-protein] reductase (NADPH) activity [GO:0141148] Also known as: enoyl-[acyl-carrier-protein] reductase activity, enoyl-ACP reductase activity, enoyl-[acyl-carrier protein] reductase activity, enoyl-[acyl-carrier-protein] reductase activity (NAD(P)H), enoyl-acyl carrier protein reductase Sources: GOC:rb